{
  "gene_symbol": "ARHGEF38",
  "term_label": "cytoplasm",
  "gene": "UniProtKB:Q9NXL2",
  "gene_name": "Rho guanine nucleotide exchange factor 38",
  "term_id": "GO:0005737"
}